{
  "term_id": "UNKNOWN:0002",
  "term_label": "Unknown biological process",
  "gene_name": "Leucine-rich repeat, immunoglobulin-like domain and transmembrane domain-containing protein 2",
  "gene_symbol": "LRIT2",
  "gene": "UniProtKB:A6NDA9"
}